positive regulation of axon extension involved in axon guidance [GO:0048842] (BP) Sources: GOC:devbiol Definition: Any process that activates, maintains or increases the frequency, rate or extent of axon extension involved in axon guidance. Also known as: up regulation of axon extension involved in axon guidance, up-regulation of axon extension involved in axon guidance, upregulation of axon extension involved in axon guidance, activation of axon extension involved in axon guidance, stimulation of axon extension involved in axon guidance Relationships: is_a positive regulation of axon extension [GO:0045773]; is a type of GO:0048841; is_a positive regulation of chemotaxis [GO:0050921]; positively regulates axon extension involved in axon guidance [GO:0048846]